{
  "term_label": "DNA-binding transcription factor activity",
  "term_id": "GO:0003700",
  "gene_symbol": "ZNF382",
  "gene": "UniProtKB:Q96SR6",
  "gene_name": "Zinc finger protein 382"
}